{
  "gene": "UniProtKB:C9JVI0",
  "gene_name": "Ubiquitin carboxyl-terminal hydrolase 17-like protein 11",
  "gene_symbol": "USP17L11",
  "term_id": "GO:0031647",
  "term_label": "regulation of protein stability"
}